{
  "gene": "UniProtKB:Q5J5C9",
  "term_label": "killing of cells of another organism",
  "gene_symbol": "DEFB121",
  "term_id": "GO:0031640",
  "gene_name": "Beta-defensin 121"
}